xyloglucan 6-xylosyltransferase activity [GO:0033843] (molecular function) Relationships: is a type of xylosyltransferase activity [GO:0042285] Also known as: UDP-D-xylose:xyloglucan 1,6-alpha-D-xylosyltransferase activity, uridine diphosphoxylose-xyloglucan 6alpha-xylosyltransferase activity, xyloglucan 6-alpha-D-xylosyltransferase activity Definition: Catalysis of the transfer of an alpha-D-xylosyl residue from UDP-D-xylose to a glucose residue in xyloglucan, forming an alpha-1,6-D-xylosyl-D-glucose linkage. Sources: EC:2.4.2.39